positive regulation of muscle contraction [GO:0045933] (biological process) Also known as: up regulation of muscle contraction, up-regulation of muscle contraction, upregulation of muscle contraction, activation of muscle contraction, stimulation of muscle contraction Relationships: is a type of regulation of muscle contraction [GO:0006937]; is_a positive regulation of multicellular organismal process [GO:0051240]; positively regulates muscle contraction [GO:0006936] Subtypes: positive regulation of smooth muscle contraction [GO:0045987], GO:0045989 Sources: GOC:go_curators Definition: Any process that activates or increases the frequency, rate or extent of muscle contraction.